{
  "term_label": "negative regulation of Ras protein signal transduction",
  "gene_name": "Protein sprouty homolog 4",
  "term_id": "GO:0046580",
  "gene_symbol": "SPRY4",
  "gene": "UniProtKB:Q9C004"
}